{
  "term_label": "membrane",
  "gene_name": "Vacuole membrane protein 1",
  "gene_symbol": "VMP1",
  "gene": "UniProtKB:Q96GC9",
  "term_id": "GO:0016020"
}